protein modification by small protein removal [GO:0070646] (biological process) Relationships: is a type of protein modification by small protein conjugation or removal [GO:0070647] Subtypes: protein deneddylation [GO:0000338], GO:0016579, protein desumoylation [GO:0016926] Definition: A protein modification process in which one or more covalently attached groups of a small protein, such as ubiquitin or a ubiquitin-like protein, are removed from a target protein. Sources: GOC:mah